NADH pyrophosphatase activity [GO:0035529] (molecular function) Definition: Catalysis of the reaction: NADH + H2O = AMP + NMNH + 2 H+. Also known as: NADH diphosphatase activity, NADH pyrophosphohydrolase activity Relationships: is a type of dinucleotide phosphatase activity [GO:0004551] References: PMID:12399474, PMID:20181750 Sources: RHEA:48868